{
  "term_label": "sperm flagellum",
  "term_id": "GO:0036126",
  "gene_symbol": "LYZL6",
  "gene_name": "Lysozyme-like protein 6",
  "gene": "UniProtKB:O75951"
}